{
  "term_label": "positive regulation of synapse assembly",
  "gene_symbol": "SRPX2",
  "term_id": "GO:0051965",
  "gene_name": "Sushi repeat-containing protein SRPX2",
  "gene": "UniProtKB:O60687"
}